{
  "gene_symbol": "UCHL3",
  "gene": "UniProtKB:P15374",
  "term_label": "protein catabolic process",
  "term_id": "GO:0030163",
  "gene_name": "Ubiquitin carboxyl-terminal hydrolase isozyme L3"
}